{
  "gene": "UniProtKB:P05090",
  "gene_name": "Apolipoprotein D",
  "term_label": "response to reactive oxygen species",
  "term_id": "GO:0000302",
  "gene_symbol": "APOD"
}